{
  "term_label": "ubiquitin-like ligase-substrate adaptor activity",
  "gene_name": "PRAME family member 15",
  "term_id": "GO:1990756",
  "gene_symbol": "PRAMEF15",
  "gene": "UniProtKB:P0DUQ1"
}